{
  "term_id": "GO:0055090",
  "gene_name": "Apolipoprotein A-V",
  "term_label": "acylglycerol homeostasis",
  "gene_symbol": "APOA5",
  "gene": "UniProtKB:Q6Q788"
}